{
  "term_id": "UNKNOWN:0002",
  "gene_symbol": "GIG44",
  "term_label": "Unknown biological process",
  "gene": "UniProtKB:P09565",
  "gene_name": "Putative insulin-like growth factor 2-associated protein"
}